4 iron, 3 sulfur cluster binding [GO:1990655] (molecular function) Definition: Binding to a 4 iron, 3 sulfur (4Fe-3S) cluster, an uncommon iron-sulfur cluster with unique properties found in oxygen-tolerant Ni-Fe hydrogenases of various bacteria. Relationships: is a type of iron-sulfur cluster binding [GO:0051536] Also known as: 4Fe-3S cluster binding References: PMID:23267108 Sources: GOC:am